{
  "gene_name": "Immunoglobulin heavy variable 1-3",
  "gene": "UniProtKB:A0A0C4DH29",
  "term_label": "immunoglobulin mediated immune response",
  "gene_symbol": "IGHV1-3",
  "term_id": "GO:0016064"
}